{
  "term_id": "GO:0043627",
  "term_label": "response to estrogen",
  "gene_name": "Zinc finger protein 366",
  "gene_symbol": "ZNF366",
  "gene": "UniProtKB:Q8N895"
}